{
  "gene_name": "Phosphatidylinositol 4-phosphate 3-kinase C2 domain-containing subunit beta",
  "gene": "UniProtKB:O00750",
  "term_id": "GO:0005886",
  "term_label": "plasma membrane",
  "gene_symbol": "PIK3C2B"
}